{
  "gene_symbol": "FBXW7",
  "gene_name": "F-box_WD repeat-containing protein 7",
  "term_label": "cytoplasm",
  "term_id": "GO:0005737",
  "gene": "UniProtKB:Q969H0"
}